{
  "gene_symbol": "HMSD",
  "term_id": "UNKNOWN:0001",
  "term_label": "Unknown molecular function",
  "gene_name": "Serpin-like protein HMSD",
  "gene": "UniProtKB:A8MTL9"
}